{
  "gene": "UniProtKB:Q9H7Z6",
  "gene_symbol": "KAT8",
  "term_label": "MSL complex",
  "gene_name": "Histone acetyltransferase KAT8",
  "term_id": "GO:0072487"
}